pyruvate metabolic process [GO:0006090] (BP) Definition: The chemical reactions and pathways involving pyruvate, 2-oxopropanoate. Relationships: is a type of monocarboxylic acid metabolic process [GO:0032787] Sources: GOC:go_curators Subtypes: pyruvate decarboxylation to acetyl-CoA [GO:0006086], glycolytic process [GO:0006096], lactate biosynthetic process from pyruvate [GO:0019244], L-alanine biosynthetic process from pyruvate [GO:0019272], GO:0019450, GO:0019617, GO:0042866, pyruvate catabolic process [GO:0042867], glycerol biosynthetic process from pyruvate [GO:0046327], Entner-Doudoroff pathway [GO:0061678], glucose catabolic process to pyruvate [GO:0061718], GO:0061722 Also known as: pyruvate metabolism, pyruvate dehydrogenase bypass